negative regulation of apoptotic process involved in metanephric nephron tubule development [GO:1900218] (biological process) Also known as: down regulation of apoptotic cell death of metanephric nephron tubule development, down regulation of apoptotic process involved in metanephric nephron tubule development, down regulation of apoptotic process of metanephric nephron tubule development, down regulation of apoptotic programmed cell death of metanephric nephron tubule development, down regulation of programmed cell death by apoptosis of metanephric nephron tubule development, down-regulation of apoptotic cell death of metanephric nephron tubule development, down-regulation of apoptotic process involved in metanephric nephron tubule development, down-regulation of apoptotic process of metanephric nephron tubule development, down-regulation of apoptotic programmed cell death of metanephric nephron tubule development, down-regulation of programmed cell death by apoptosis of metanephric nephron tubule development, downregulation of apoptotic cell death of metanephric nephron tubule development, downregulation of apoptotic process involved in metanephric nephron tubule development, downregulation of apoptotic process of metanephric nephron tubule development, downregulation of apoptotic programmed cell death of metanephric nephron tubule development, downregulation of programmed cell death by apoptosis of metanephric nephron tubule development, inhibition of apoptotic cell death of metanephric nephron tubule development, inhibition of apoptotic process of metanephric nephron tubule development, inhibition of apoptotic programmed cell death of metanephric nephron tubule development, inhibition of programmed cell death by apoptosis of metanephric nephron tubule development, negative regulation of apoptotic cell death of metanephric nephron tubule development, negative regulation of apoptotic process of metanephric nephron tubule development, negative regulation of apoptotic programmed cell death of metanephric nephron tubule development, negative regulation of programmed cell death by apoptosis of metanephric nephron tubule development, down regulation of apoptosis of metanephric nephron tubule development, down regulation of apoptotic program of metanephric nephron tubule development, down regulation of type I programmed cell death of metanephric nephron tubule development, down-regulation of apoptosis of metanephric nephron tubule development, down-regulation of apoptotic program of metanephric nephron tubule development, down-regulation of type I programmed cell death of metanephric nephron tubule development, downregulation of apoptosis of metanephric nephron tubule development, downregulation of apoptotic program of metanephric nephron tubule development, downregulation of type I programmed cell death of metanephric nephron tubule development, inhibition of apoptosis of metanephric nephron tubule development, inhibition of apoptotic process involved in metanephric nephron tubule development, inhibition of apoptotic program of metanephric nephron tubule development, inhibition of type I programmed cell death of metanephric nephron tubule development, negative regulation of apoptosis of metanephric nephron tubule development, negative regulation of apoptotic program of metanephric nephron tubule development, negative regulation of type I programmed cell death of metanephric nephron tubule development, down regulation of signaling (initiator) caspase activity of metanephric nephron tubule development, down-regulation of signaling (initiator) caspase activity of metanephric nephron tubule development, downregulation of signaling (initiator) caspase activity of metanephric nephron tubule development, inhibition of signaling (initiator) caspase activity of metanephric nephron tubule development, negative regulation of signaling (initiator) caspase activity of metanephric nephron tubule development Definition: Any process that stops, prevents or reduces the frequency, rate or extent of apoptotic process involved in metanephric nephron tubule development. References: PMID:17314325 Sources: GOC:TermGenie, GOC:mtg_kidney_jan10, GOC:yaf Relationships: is a type of regulation of apoptotic process involved in metanephric nephron tubule development [GO:1900217]; is a type of negative regulation of apoptotic process involved in development [GO:1904746]; negatively regulates apoptotic process involved in metanephric nephron tubule development [GO:1900205]